{
  "gene_name": "Insulin-like growth factor 1 receptor",
  "term_id": "GO:0071333",
  "gene": "UniProtKB:P08069",
  "term_label": "cellular response to glucose stimulus",
  "gene_symbol": "IGF1R"
}